{
  "gene_name": "Psoriasis susceptibility 1 candidate gene 2 protein",
  "gene_symbol": "PSORS1C2",
  "term_label": "Unknown molecular function",
  "term_id": "UNKNOWN:0001",
  "gene": "UniProtKB:Q9UIG4"
}